negative regulation of vacuolar transport [GO:1903336] (biological process) Subtypes: negative regulation of protein targeting to vacuolar membrane [GO:1900484], GO:1902823, GO:1904052 Relationships: is a type of GO:0032387; is a type of regulation of vacuolar transport [GO:1903335]; negatively regulates GO:0007034 Also known as: down regulation of vacuolar transport, down-regulation of vacuolar transport, downregulation of vacuolar transport, inhibition of vacuolar transport Definition: Any process that stops, prevents or reduces the frequency, rate or extent of vacuolar transport. Sources: GOC:TermGenie, GOC:vw, GO_REF:0000058